{
  "gene_symbol": "TMEM171",
  "gene_name": "Transmembrane protein 171",
  "term_label": "Unknown cellular component",
  "term_id": "UNKNOWN:0003",
  "gene": "UniProtKB:Q8WVE6"
}